trigeminal nerve maturation [GO:0021635] (biological process) Sources: GOC:cls, GOC:dgh, GOC:dph, GOC:jid, GO_REF:0000021 Relationships: is a type of GO:0021605; is part of trigeminal nerve development [GO:0021559] Definition: A developmental process, independent of morphogenetic (shape) change, that is required for the trigeminal nerve to attain its fully functional state. The trigeminal nerve is composed of three large branches. They are the ophthalmic (V1, sensory), maxillary (V2, sensory) and mandibular (V3, motor and sensory) branches. The sensory ophthalmic branch travels through the superior orbital fissure and passes through the orbit to reach the skin of the forehead and top of the head. The maxillary nerve contains sensory branches that reach the pterygopalatine fossa via the inferior orbital fissure (face, cheek and upper teeth) and pterygopalatine canal (soft and hard palate, nasal cavity and pharynx). The motor part of the mandibular branch is distributed to the muscles of mastication, the mylohyoid muscle and the anterior belly of the digastric. The mandibular nerve also innervates the tensor veli palatini and tensor tympani muscles. The sensory part of the mandibular nerve is composed of branches that carry general sensory information from the mucous membranes of the mouth and cheek, anterior two-thirds of the tongue, lower teeth, skin of the lower jaw, side of the head and scalp and meninges of the anterior and middle cranial fossae. Also known as: CN V maturation